{
  "gene_name": "Dedicator of cytokinesis protein 4",
  "term_label": "cytoplasm",
  "gene": "UniProtKB:Q8N1I0",
  "term_id": "GO:0005737",
  "gene_symbol": "DOCK4"
}